{
  "gene_symbol": "COPZ2",
  "gene": "UniProtKB:Q9P299",
  "gene_name": "Coatomer subunit zeta-2",
  "term_id": "GO:0006890",
  "term_label": "retrograde vesicle-mediated transport, Golgi to endoplasmic reticulum"
}